apoptotic process involved in mammary gland involution [GO:0060057] (biological process) Sources: GOC:dph, GOC:mtg_apoptosis Regulation: RO_0002213 by positive regulation of apoptotic process involved in mammary gland involution [GO:0060058] Definition: Any apoptotic process that triggers the activity of proteolytic caspases whose actions dismantle the mammary epithelial cells resulting in their programmed cell death. Relationships: is a type of GO:0060561; is part of mammary gland involution [GO:0060056] Also known as: apoptosis involved in mammary gland involution